acetylserotonin O-methyltransferase activity [GO:0017096] (MF) Sources: EC:2.1.1.4 Relationships: is a type of O-methyltransferase activity [GO:0008171]; is a type of S-adenosylmethionine-dependent methyltransferase activity [GO:0008757] Definition: Catalysis of the reaction: S-adenosyl-L-methionine + N-acetylserotonin = S-adenosyl-L-homocysteine + melatonin. Melatonin is also known as N-acetyl-5-methoxytryptamine. Also known as: N-acetylserotonin O-methyltransferase activity, S-adenosyl-L-methionine:N-acetylserotonin O-methyltransferase activity, acetylserotonin methyltransferase activity, hydroxyindole O-methyltransferase activity, hydroxyindole methyltransferase activity